Fc-gamma receptor I complex binding [GO:0034988] (molecular function) Definition: Binding to one or more specific sites on the Fc-gamma receptor I complex. The complex functions primarily as an activating receptor for IgG. Relationships: is a type of immunoglobulin receptor binding [GO:0034987]; is a type of protein-containing complex binding [GO:0044877] Sources: GOC:BHF, GOC:vk